{
  "gene_symbol": "FANCB",
  "gene_name": "Fanconi anemia group B protein",
  "term_id": "GO:2000042",
  "gene": "UniProtKB:Q8NB91",
  "term_label": "negative regulation of double-strand break repair via homologous recombination"
}